{
  "gene": "UniProtKB:Q96EX1",
  "term_label": "Unknown biological process",
  "gene_name": "Small integral membrane protein 12",
  "term_id": "UNKNOWN:0002",
  "gene_symbol": "SMIM12"
}